{
  "term_label": "dendrite self-avoidance",
  "term_id": "GO:0070593",
  "gene_name": "Contactin-2",
  "gene_symbol": "CNTN2",
  "gene": "UniProtKB:Q02246"
}